protein N-terminal-methionine acetyltransferase activity [GO:0120518] (molecular function) Sources: RHEA:75239 Definition: Catalysis of the reaction: acetyl-CoA + N-terminal L-methionyl-[protein] = CoA + H+ + N-terminal N(alpha)-acetyl-L-methionyl-[protein]. Also known as: peptide-methionine-alpha-N-acetyltransferase activity Relationships: is a type of protein-N-terminal amino-acid acetyltransferase activity [GO:0004596]